{
  "gene_symbol": "NCS1",
  "term_id": "GO:0005509",
  "gene": "UniProtKB:P62166",
  "term_label": "calcium ion binding",
  "gene_name": "Neuronal calcium sensor 1"
}